{
  "gene_symbol": "TNFRSF19",
  "gene": "UniProtKB:Q9NS68",
  "term_label": "positive regulation of JNK cascade",
  "gene_name": "Tumor necrosis factor receptor superfamily member 19",
  "term_id": "GO:0046330"
}